{
  "term_id": "GO:0048024",
  "gene": "UniProtKB:Q86U06",
  "gene_name": "Probable RNA-binding protein 23",
  "term_label": "regulation of mRNA splicing, via spliceosome",
  "gene_symbol": "RBM23"
}